{
  "gene": "UniProtKB:Q9NX58",
  "term_label": "DNA binding",
  "term_id": "GO:0003677",
  "gene_name": "Cell growth-regulating nucleolar protein",
  "gene_symbol": "LYAR"
}